{
  "gene_name": "Solute carrier family 35 member G2",
  "term_id": "UNKNOWN:0002",
  "gene_symbol": "SLC35G2",
  "gene": "UniProtKB:Q8TBE7",
  "term_label": "Unknown biological process"
}